{
  "gene": "UniProtKB:Q8NH87",
  "term_label": "Unknown cellular component",
  "term_id": "UNKNOWN:0003",
  "gene_symbol": "OR9G1",
  "gene_name": "Olfactory receptor 9G1"
}